establishment of competence for transformation [GO:0030420] (biological process) Relationships: is a type of cellular response to stimulus [GO:0051716]; is part of DNA-mediated transformation [GO:0009294] Regulation: regulated by regulation of establishment of competence for transformation [GO:0045304]; RO_0002212 by negative regulation of establishment of competence for transformation [GO:0045808]; positively regulated by GO:0045809 Definition: The process in which a naturally transformable bacterium acquires the ability to take up exogenous DNA. This term should be applied only to naturally transformable bacteria, and should not be used in the context of artificially induced bacterial transformation. Sources: GOC:mah, ISBN:1555811027